{
  "term_label": "positive regulation of gene expression",
  "gene": "UniProtKB:Q6DKI2",
  "term_id": "GO:0010628",
  "gene_symbol": "LGALS9C",
  "gene_name": "Galectin-9C"
}